{
  "term_id": "GO:0022857",
  "gene_symbol": "SFXN4",
  "gene": "UniProtKB:Q6P4A7",
  "gene_name": "Sideroflexin-4",
  "term_label": "transmembrane transporter activity"
}